{
  "gene_symbol": "LILRB3",
  "term_id": "GO:0005886",
  "term_label": "plasma membrane",
  "gene_name": "Leukocyte immunoglobulin-like receptor subfamily B member 3",
  "gene": "UniProtKB:O75022"
}